{
  "gene_symbol": "SLC43A2",
  "term_id": "GO:0015179",
  "term_label": "L-amino acid transmembrane transporter activity",
  "gene_name": "Large neutral amino acids transporter small subunit 4",
  "gene": "UniProtKB:Q8N370"
}